{
  "gene_name": "Fatty acid 2-hydroxylase",
  "term_label": "endoplasmic reticulum",
  "term_id": "GO:0005783",
  "gene": "UniProtKB:Q7L5A8",
  "gene_symbol": "FA2H"
}